{
  "gene": "UniProtKB:Q6PEW1",
  "gene_symbol": "ZCCHC12",
  "term_id": "GO:0005634",
  "gene_name": "Zinc finger CCHC domain-containing protein 12",
  "term_label": "nucleus"
}